medium-chain fatty acid omega-1 hydroxylase activity [GO:0120503] (molecular function) Definition: Catalysis of the reaction: an (omega-1)-ethyl medium-chain fatty acid + O2 + reduced [NADPH-hemoprotein reductase] = an (omega-1)-hydroxy-medium-chain fatty acid + H+ + H2O + oxidized [NADPH-hemoprotein reductase. A medium-chain fatty acid has an aliphatic tail containing 6 to 12 carbons. References: PMID:35934685 Note: While there is not universal consensus on the lengths of short-, medium-, long- and very-long-chain fatty acids, the GO uses the definitions in ChEBI (see CHEBI:26666, CHEBI:59554, CHEBI:15904 and CHEBI:27283). Relationships: is a type of GO:0120502